{
  "term_label": "plasma membrane",
  "term_id": "GO:0005886",
  "gene_name": "Voltage-gated hydrogen channel 1",
  "gene_symbol": "HVCN1",
  "gene": "UniProtKB:Q96D96"
}